proboscis morphogenesis [GO:0048734] (biological process) Sources: GOC:jid, GOC:rc Definition: The process in which the anatomical structures of the proboscis are generated and organized. The proboscis is the trunk-like extension of the mouthparts on the adult head. Relationships: is a type of animal organ morphogenesis [GO:0009887]; is part of proboscis development [GO:0048728]